negative regulation of cerebellar granule cell precursor proliferation [GO:0021941] (biological process) Relationships: is a type of regulation of cerebellar granule cell precursor proliferation [GO:0021936]; is a type of negative regulation of neural precursor cell proliferation [GO:2000178]; negatively regulates GO:0021930 Definition: The process that stops, prevents or reduces the rate or extent of granule cell precursor proliferation. Also known as: down regulation of granule cell precursor proliferation, down-regulation of granule cell precursor proliferation, downregulation of granule cell precursor proliferation, inhibition of granule cell precursor proliferation References: PMID:15157725 Sources: GOC:cls, GOC:dgh, GOC:dph, GOC:jid, GO_REF:0000021